olfactory bulb axon guidance [GO:0071678] (BP) Sources: GOC:BHF, GOC:mah Also known as: olfactory bulb axon pathfinding Definition: The process in which the migration of an axon growth cone of a neuron in the olfactory bulb is directed to its target in the brain in response to a combination of attractive and repulsive cues. Relationships: is a type of axon guidance [GO:0007411]